{
  "gene": "UniProtKB:P20671",
  "term_id": "GO:0031507",
  "gene_name": "Histone H2A type 1-D",
  "term_label": "heterochromatin formation",
  "gene_symbol": "H2AC7"
}